{
  "gene_name": "Calcium-responsive transcription factor",
  "term_label": "DNA-binding transcription factor activity, RNA polymerase II-specific",
  "term_id": "GO:0000981",
  "gene_symbol": "CARF",
  "gene": "UniProtKB:Q8N187"
}